{
  "gene_symbol": "LYSMD1",
  "gene_name": "LysM and putative peptidoglycan-binding domain-containing protein 1",
  "term_label": "Unknown cellular component",
  "term_id": "UNKNOWN:0003",
  "gene": "UniProtKB:Q96S90"
}